{
  "gene_symbol": "TMEM201",
  "term_id": "GO:0031965",
  "gene": "UniProtKB:Q5SNT2",
  "gene_name": "Transmembrane protein 201",
  "term_label": "nuclear membrane"
}